{
  "gene_name": "Protein eva-1 homolog A",
  "term_label": "Unknown cellular component",
  "gene": "UniProtKB:Q9H8M9",
  "term_id": "UNKNOWN:0003",
  "gene_symbol": "EVA1A"
}